lateral mesoderm structural organization [GO:0048381] (biological process) Definition: The process that contributes to the act of creating the structural organization of the lateral mesoderm. This process pertains to the physical shaping of a rudimentary structure. Sources: GOC:jid Also known as: lateral mesoderm structural organisation, lateral plate mesoderm structural organization Relationships: is_a mesoderm structural organization [GO:0048338]; is part of lateral mesoderm morphogenesis [GO:0048369]